{
  "term_id": "GO:0031463",
  "gene_symbol": "TNFAIP1",
  "gene": "UniProtKB:Q13829",
  "term_label": "Cul3-RING ubiquitin ligase complex",
  "gene_name": "BTB_POZ domain-containing adapter for CUL3-mediated RhoA degradation protein 2"
}